{
  "gene_symbol": "FBXO30",
  "gene_name": "F-box only protein 30",
  "term_id": "UNKNOWN:0001",
  "term_label": "Unknown molecular function",
  "gene": "UniProtKB:Q8TB52"
}